{
  "term_label": "Unknown cellular component",
  "gene_symbol": "UNQ6190_PRO20217",
  "gene": "UniProtKB:Q6UXQ8",
  "term_id": "UNKNOWN:0003",
  "gene_name": "Putative uncharacterized protein UNQ6190_PRO20217"
}